{
  "gene_name": "Netrin receptor DCC",
  "gene": "UniProtKB:P43146",
  "term_id": "GO:0005886",
  "term_label": "plasma membrane",
  "gene_symbol": "DCC"
}